{
  "gene_name": "Serine--tRNA ligase, cytoplasmic",
  "term_id": "GO:0002181",
  "term_label": "cytoplasmic translation",
  "gene_symbol": "SARS1",
  "gene": "UniProtKB:P49591"
}